{
  "term_id": "GO:0001836",
  "gene_name": "Bcl-2-like protein 10",
  "term_label": "release of cytochrome c from mitochondria",
  "gene": "UniProtKB:Q9HD36",
  "gene_symbol": "BCL2L10"
}